{
  "gene_name": "Epididymal protein 13",
  "term_label": "Unknown molecular function",
  "term_id": "UNKNOWN:0001",
  "gene": "UniProtKB:A0A1B0GTR0",
  "gene_symbol": "EDDM13"
}